{
  "gene_name": "Peptidyl-prolyl cis-trans isomerase G",
  "gene_symbol": "PPIG",
  "term_label": "nucleus",
  "term_id": "GO:0005634",
  "gene": "UniProtKB:Q13427"
}